hepatic stellate cell migration [GO:0061868] (biological process) Regulation: regulated by regulation of hepatic stellate cell migration [GO:0061869]; positively regulated by positive regulation of hepatic stellate cell migration [GO:0061870]; negatively regulated by negative regulation of hepatic stellate cell migration [GO:0061871] Relationships: is a type of fibroblast migration [GO:0010761] References: PMID:24204762 Definition: The orderly movement of a hepatic stellate cell from one site to another.